{
  "gene_name": "Protein spinster homolog 3",
  "gene_symbol": "SPNS3",
  "gene": "UniProtKB:Q6ZMD2",
  "term_label": "membrane",
  "term_id": "GO:0016020"
}